{
  "gene_symbol": "SH3TC2",
  "gene": "UniProtKB:Q8TF17",
  "gene_name": "SH3 domain and tetratricopeptide repeat-containing protein 2",
  "term_label": "regulation of ERBB signaling pathway",
  "term_id": "GO:1901184"
}